{
  "term_id": "UNKNOWN:0002",
  "gene_name": "Protein FAM240A",
  "gene": "UniProtKB:A0A1B0GVK7",
  "gene_symbol": "FAM240A",
  "term_label": "Unknown biological process"
}